{
  "term_label": "intracellular protein transport",
  "gene_name": "ADP-ribosylation factor-related protein 1",
  "term_id": "GO:0006886",
  "gene_symbol": "ARFRP1",
  "gene": "UniProtKB:Q13795"
}